cone photoresponse recovery [GO:0036368] (biological process) References: PMID:16039565, PMID:22802362 Sources: GOC:gap Also known as: cone response recovery, cone phototransduction termination Definition: The processes required for a cone photoreceptor to recover, following light activation, so that it can respond to a subsequent light stimulus. Cone recovery requires the shutoff of active participants in the phototransduction cascade, including the visual pigment and downstream signal transducers. Relationships: is a type of response to light stimulus [GO:0009416]